24-methylenelophenol methyl oxidase activity [GO:0102177] (molecular function) Relationships: is a type of oxidoreductase activity, acting on paired donors, with incorporation or reduction of molecular oxygen, NAD(P)H as one donor, and incorporation of one atom of oxygen [GO:0016709] Definition: Catalysis of the reaction: 24-methylenelophenol + O2 + NADH + H+ = 4alpha-hydroxymethyl-ergosta-7,24(241)-dien-3beta-ol + NAD + H2O. References: PMID:11707264 Sources: GOC:pz, RHEA:58872